negative regulation of lipoprotein lipid oxidation [GO:0060588] (biological process) Relationships: is a type of negative regulation of lipoprotein oxidation [GO:0034443]; is a type of negative regulation of lipid metabolic process [GO:0045833]; is a type of regulation of lipoprotein lipid oxidation [GO:0060587]; RO_0002212 lipoprotein lipid oxidation [GO:0034439] Definition: Any process that decreases the rate, frequency or extent of lipoprotein lipid oxidation. Lipoprotein lipid oxidation is the modification of a lipoprotein by oxidation of the lipid group. Sources: GOC:BHF, GOC:dph, GOC:tb